{
  "gene_name": "Nck-associated protein 1",
  "gene": "UniProtKB:Q9Y2A7",
  "term_id": "GO:0000902",
  "gene_symbol": "NCKAP1",
  "term_label": "cell morphogenesis"
}